{
  "gene_symbol": "ADRA2C",
  "term_label": "epinephrine binding",
  "gene": "UniProtKB:P18825",
  "term_id": "GO:0051379",
  "gene_name": "Alpha-2C adrenergic receptor"
}